{
  "gene": "UniProtKB:Q05BV3",
  "gene_symbol": "EML5",
  "gene_name": "Echinoderm microtubule-associated protein-like 5",
  "term_label": "Unknown biological process",
  "term_id": "UNKNOWN:0002"
}